{
  "term_label": "RNA polymerase II cis-regulatory region sequence-specific DNA binding",
  "gene_name": "Prospero homeobox protein 2",
  "term_id": "GO:0000978",
  "gene_symbol": "PROX2",
  "gene": "UniProtKB:Q3B8N5"
}